protein phosphatase activator activity [GO:0072542] (molecular function) Relationships: is a type of phosphatase activator activity [GO:0019211]; is a type of protein phosphatase regulator activity [GO:0019888]; positively regulates phosphoprotein phosphatase activity [GO:0004721] Also known as: protein phosphatase 2 activator activity, protein phosphatase type 1 activator activity, protein phosphatase type 2A activator activity Subtypes: protein tyrosine phosphatase activator activity [GO:0008160] Sources: GOC:mah Definition: Binds to and increases the activity of a protein phosphatase.